bis(5'-nucleosidyl) oligophosphate biosynthetic process [GO:0015957] (biological process) Definition: The chemical reactions and pathways resulting in the formation of a bis(5'-nucleosidyl) oligophosphate, a compound formed of two nucleosides joined together through their 5' carbons by a chain of phosphate molecules. Relationships: is a type of nucleotide biosynthetic process [GO:0009165] Also known as: bis(5'-nucleosidyl) oligophosphate anabolism, bis(5'-nucleosidyl) oligophosphate biosynthesis, bis(5'-nucleosidyl) oligophosphate formation, bis(5'-nucleosidyl) oligophosphate synthesis References: PMID:10970777 Sources: GOC:mah